{
  "gene_symbol": "DGAT2",
  "term_id": "GO:0004144",
  "gene": "UniProtKB:Q96PD7",
  "term_label": "diacylglycerol O-acyltransferase activity",
  "gene_name": "Diacylglycerol O-acyltransferase 2"
}